positive regulation of core promoter binding [GO:1904798] (biological process) Relationships: is a type of positive regulation of transcription regulatory region DNA binding [GO:2000679]; positively regulates core promoter sequence-specific DNA binding [GO:0001046] Also known as: up regulation of core promoter binding, up-regulation of core promoter binding, upregulation of core promoter binding, activation of core promoter binding References: PMID:22723415 Sources: GOC:BHF, GOC:BHF_telomere, GOC:TermGenie, GOC:nc, GO_REF:0000059 Definition: Any process that activates or increases the frequency, rate or extent of core promoter binding.